{
  "gene": "UniProtKB:Q9BQJ4",
  "gene_name": "Transmembrane protein 47",
  "term_id": "GO:0098609",
  "term_label": "cell-cell adhesion",
  "gene_symbol": "TMEM47"
}